ligand-gated monoatomic cation channel activity [GO:0099094] (MF) Also known as: ligand-gated cation channel activity Relationships: is a type of monoatomic cation channel activity [GO:0005261]; is a type of GO:0015276 Subtypes: extracellularly ATP-gated monoatomic cation channel activity [GO:0004931], intracellularly cyclic nucleotide-activated monoatomic cation channel activity [GO:0005221], calcium-activated cation channel activity [GO:0005227], GO:0005228, inward rectifier potassium channel activity [GO:0005242], ligand-gated sodium channel activity [GO:0015280], GO:0022848, serotonin-gated monoatomic cation channel activity [GO:0022850], mitochondrial ATP-gated potassium channel activity [GO:0062156], chloride-activated potassium channel activity [GO:0070089], glycine betaine-activated nonselective monoatomic cation channel activity [GO:0090686], GO:0097682, ligand-gated calcium channel activity [GO:0099604], glycine-gated cation channel activity [GO:0160212] Sources: GOC:mtg_transport, ISBN:0815340729 Definition: Enables the transmembrane transfer of an inorganic cation by a channel that opens when a specific ligand has been bound by the channel complex or one of its constituent parts.